motogenic signaling involved in postnatal olfactory bulb interneuron migration [GO:0021837] (BP) Definition: The signaling that results in the stimulation of cell movement in the rostral migratory stream. Also known as: motogenic signalling involved in postnatal olfactory bulb interneuron migration References: PMID:12626695 Sources: GOC:cls, GOC:dgh, GOC:dph, GOC:jid, GO_REF:0000021 Relationships: is a type of GO:0007154; is a type of signaling [GO:0023052]; is part of GO:0021827